{
  "gene": "UniProtKB:Q9Y615",
  "term_label": "Unknown biological process",
  "gene_symbol": "ACTL7A",
  "term_id": "UNKNOWN:0002",
  "gene_name": "Actin-like protein 7A"
}